{
  "term_label": "nucleus",
  "gene_name": "Melanoma-associated antigen 6",
  "gene_symbol": "MAGEA6",
  "term_id": "GO:0005634",
  "gene": "UniProtKB:P43360"
}